{
  "gene_symbol": "ARF1",
  "gene": "UniProtKB:P84077",
  "gene_name": "ADP-ribosylation factor 1",
  "term_id": "GO:0016192",
  "term_label": "vesicle-mediated transport"
}